{
  "term_label": "skeletal system development",
  "gene": "UniProtKB:Q9NX62",
  "term_id": "GO:0001501",
  "gene_name": "Golgi-resident adenosine 3',5'-bisphosphate 3'-phosphatase",
  "gene_symbol": "BPNT2"
}